sphingolipid 8-(E/Z)-desaturase activity [GO:0052631] (molecular function) Definition: Catalysis of the reaction: an N-acyl-(4R)-4-hydroxysphinganine + 2 Fe(II)-[cytochrome b5] + 2 H+ + O2 = a (4R,8E)-4-hydroxysphingenine ceramide + 2 Fe(III)-[cytochrome b5] + 2 H2O or an N-acyl-(4R)-4-hydroxysphinganine + 2 Fe(II)-[cytochrome b5] + 2 H+ + O2 = (4R,8Z)-4-hydroxysphing-8-enine ceramide + 2 Fe(III)-[cytochrome b5] + 2 H2O. This results in the formation of a double bond between C8 and C9 of the long chain base of a sphingolipid. References: PMID:17600137, PMID:9786850 Sources: EC:1.14.19.29 Relationships: is_a oxidoreductase activity, acting on paired donors, with oxidation of a pair of donors resulting in the reduction of molecular oxygen to two molecules of water [GO:0016717] Also known as: 8 fatty acid desaturase, 8-sphingolipid desaturase, sphingolipid delta-8 desaturase activity